{
  "gene_name": "Serine_threonine-protein phosphatase 6 regulatory subunit 1",
  "gene_symbol": "PPP6R1",
  "term_id": "GO:0005829",
  "gene": "UniProtKB:Q9UPN7",
  "term_label": "cytosol"
}